deoxyribonucleoside diphosphate catabolic process [GO:0009192] (BP) Also known as: deoxyribonucleoside diphosphate breakdown, deoxyribonucleoside diphosphate catabolism, deoxyribonucleoside diphosphate degradation Subtypes: purine deoxyribonucleoside diphosphate catabolic process [GO:0009184], pyrimidine deoxyribonucleoside diphosphate catabolic process [GO:0009198] Definition: The chemical reactions and pathways resulting in the breakdown of a deoxyribonucleoside diphosphate, a compound consisting of a nucleobase linked to a deoxyribose sugar esterified with diphosphate on the sugar. Sources: GOC:go_curators, ISBN:0198506732 Relationships: is a type of nucleoside diphosphate catabolic process [GO:0009134]